{
  "gene_name": "Putative GED domain-containing protein DNM1P34",
  "gene": "UniProtKB:Q6PK57",
  "term_id": "UNKNOWN:0002",
  "gene_symbol": "DNM1P34",
  "term_label": "Unknown biological process"
}